{
  "gene": "UniProtKB:Q9HCL2",
  "term_id": "GO:0005739",
  "term_label": "mitochondrion",
  "gene_symbol": "GPAM",
  "gene_name": "Glycerol-3-phosphate acyltransferase 1, mitochondrial"
}